{
  "term_id": "GO:0005615",
  "gene_name": "Thyrotropin subunit beta",
  "gene": "UniProtKB:P01222",
  "gene_symbol": "TSHB",
  "term_label": "extracellular space"
}